{
  "gene_name": "Rho GTPase-activating protein 23",
  "term_id": "UNKNOWN:0003",
  "gene_symbol": "ARHGAP23",
  "term_label": "Unknown cellular component",
  "gene": "UniProtKB:Q9P227"
}